{
  "gene_symbol": "OR6K6",
  "gene": "UniProtKB:Q8NGW6",
  "gene_name": "Olfactory receptor 6K6",
  "term_label": "odorant binding",
  "term_id": "GO:0005549"
}